{
  "gene_symbol": "ZNF98",
  "term_label": "RNA polymerase II cis-regulatory region sequence-specific DNA binding",
  "gene": "UniProtKB:A6NK75",
  "gene_name": "Zinc finger protein 98",
  "term_id": "GO:0000978"
}